{
  "term_id": "GO:0006631",
  "term_label": "fatty acid metabolic process",
  "gene": "UniProtKB:P07108",
  "gene_symbol": "DBI",
  "gene_name": "Acyl-CoA-binding protein"
}